{
  "gene": "UniProtKB:Q8WYJ6",
  "term_id": "GO:0003924",
  "term_label": "GTPase activity",
  "gene_name": "Septin-1",
  "gene_symbol": "SEPTIN1"
}